{
  "gene_name": "Ankyrin repeat and fibronectin type-III domain-containing protein 1",
  "term_id": "GO:0000132",
  "gene_symbol": "ANKFN1",
  "gene": "UniProtKB:Q8N957",
  "term_label": "establishment of mitotic spindle orientation"
}